{
  "term_id": "GO:0008083",
  "gene_symbol": "VEGFB",
  "term_label": "growth factor activity",
  "gene_name": "Vascular endothelial growth factor B",
  "gene": "UniProtKB:P49765"
}